{
  "term_id": "GO:0000781",
  "gene_symbol": "RPA4",
  "term_label": "chromosome, telomeric region",
  "gene_name": "Replication protein A 30 kDa subunit",
  "gene": "UniProtKB:Q13156"
}